{
  "gene_name": "Small RNA 2'-O-methyltransferase",
  "term_label": "nucleus",
  "gene_symbol": "HENMT1",
  "term_id": "GO:0005634",
  "gene": "UniProtKB:Q5T8I9"
}